{
  "term_label": "innate immune response",
  "gene_name": "Zinc finger protein RFP",
  "term_id": "GO:0045087",
  "gene": "UniProtKB:P14373",
  "gene_symbol": "TRIM27"
}